{
  "term_label": "proton-transporting ATP synthase complex",
  "term_id": "GO:0045259",
  "gene_symbol": "ATP5F1B",
  "gene": "UniProtKB:P06576",
  "gene_name": "ATP synthase subunit beta, mitochondrial"
}